cellular response to homocysteine [GO:1905375] (BP) Also known as: cellular response to 2-amino-4-mercaptobutyric acid, cellular response to 2-amino-4-sulfanylbutanoic acid, cellular response to Hcy Definition: Any process that results in a change in state or activity of a cell (in terms of movement, secretion, enzyme production, gene expression, etc.) as a result of a homocysteine stimulus. References: PMID:26722473 Sources: GOC:TermGenie, GO_REF:0000071 Relationships: is a type of cellular response to amino acid stimulus [GO:0071230]; is_a cellular response to nitrogen compound [GO:1901699]; is a type of cellular response to oxygen-containing compound [GO:1901701]; is a type of response to homocysteine [GO:1905374]